{
  "gene": "UniProtKB:P28062",
  "term_label": "proteasome-mediated ubiquitin-dependent protein catabolic process",
  "term_id": "GO:0043161",
  "gene_name": "Proteasome subunit beta type-8",
  "gene_symbol": "PSMB8"
}